{
  "gene_symbol": "SECISBP2L",
  "gene": "UniProtKB:Q93073",
  "term_label": "Unknown biological process",
  "term_id": "UNKNOWN:0002",
  "gene_name": "Selenocysteine insertion sequence-binding protein 2-like"
}